{
  "gene_symbol": "TBCA",
  "term_label": "microtubule cytoskeleton",
  "gene_name": "Tubulin-specific chaperone A",
  "gene": "UniProtKB:O75347",
  "term_id": "GO:0015630"
}